{
  "gene_name": "Polyhomeotic-like protein 3",
  "term_id": "GO:0005634",
  "gene_symbol": "PHC3",
  "gene": "UniProtKB:Q8NDX5",
  "term_label": "nucleus"
}